{
  "gene": "UniProtKB:Q9NWZ3",
  "gene_name": "Interleukin-1 receptor-associated kinase 4",
  "term_label": "cytoplasm",
  "gene_symbol": "IRAK4",
  "term_id": "GO:0005737"
}